{
  "gene_symbol": "ANKRD42",
  "gene": "UniProtKB:Q8N9B4",
  "term_id": "UNKNOWN:0002",
  "term_label": "Unknown biological process",
  "gene_name": "Ankyrin repeat domain-containing protein 42"
}